benzoyl-CoA catabolic process [GO:1901788] (biological process) Definition: The chemical reactions and pathways resulting in the breakdown of benzoyl-CoA. Sources: GOC:TermGenie, GOC:yaf, MetaCyc:CENTBENZCOA-PWY, MetaCyc:P321-PWY, MetaCyc:PWY-1361 Relationships: is a type of sulfur compound catabolic process [GO:0044273]; is a type of purine-containing compound catabolic process [GO:0072523]; is a type of nucleoside phosphate catabolic process [GO:1901292]; is a type of benzoyl-CoA metabolic process [GO:1901787] Also known as: benzoyl-CoA breakdown, benzoyl-CoA catabolism, benzoyl-CoA degradation